{
  "gene": "UniProtKB:Q86Y26",
  "gene_symbol": "NUTM1",
  "term_id": "UNKNOWN:0003",
  "term_label": "Unknown cellular component",
  "gene_name": "NUT family member 1"
}